negative regulation of skeletal muscle fiber development [GO:0048744] (biological process) Definition: Any process that stops, prevents, or reduces the frequency, rate or extent of skeletal muscle fiber development. Muscle fibers are formed by the maturation of myotubes. They can be classed as slow, intermediate/fast or fast. Relationships: is a type of negative regulation of cell development [GO:0010721]; is a type of regulation of skeletal muscle fiber development [GO:0048742]; is a type of negative regulation of striated muscle cell differentiation [GO:0051154]; negatively regulates skeletal muscle fiber development [GO:0048741] Also known as: down regulation of skeletal muscle fiber development, down-regulation of skeletal muscle fiber development, downregulation of skeletal muscle fiber development, negative regulation of skeletal muscle fibre development, negative regulation of skeletal myofiber development, negative regulation of skeletal myofibre development, inhibition of skeletal muscle fiber development Sources: GOC:dph, GOC:jid, GOC:lm, GOC:mtg_muscle